regulation of floral meristem growth [GO:0010080] (biological process) Sources: GOC:tb Definition: Any process involved in maintaining the size and shape of a floral meristem. Relationships: is a type of regulation of meristem growth [GO:0010075]; is a type of regulation of reproductive process [GO:2000241]; regulates floral meristem growth [GO:0010451] Also known as: regulation of floral meristem size